{
  "gene": "UniProtKB:Q9HCE6",
  "term_label": "positive regulation of stress fiber assembly",
  "gene_symbol": "ARHGEF10L",
  "term_id": "GO:0051496",
  "gene_name": "Rho guanine nucleotide exchange factor 10-like protein"
}